{
  "gene_symbol": "STX19",
  "gene_name": "Syntaxin-19",
  "term_label": "presynaptic active zone membrane",
  "gene": "UniProtKB:Q8N4C7",
  "term_id": "GO:0048787"
}